{
  "term_id": "GO:0000977",
  "gene_name": "Achaete-scute homolog 1",
  "term_label": "RNA polymerase II transcription regulatory region sequence-specific DNA binding",
  "gene_symbol": "ASCL1",
  "gene": "UniProtKB:P50553"
}